cystine:glutamate antiporter activity [GO:0015327] (molecular function) Relationships: is a type of GO:0000099; is_a GO:0005313; is_a GO:0015297; is a type of modified amino acid transmembrane transporter activity [GO:0072349] Definition: Enables the transfer of a solute or solutes from one side of a membrane to the other according to the reaction: cystine(out) + glutamate(in) = cystine(in) + glutamate(out). Sources: TC:2.A.3.8.5